{
  "gene_symbol": "TMEM171",
  "term_label": "Unknown biological process",
  "gene": "UniProtKB:Q8WVE6",
  "gene_name": "Transmembrane protein 171",
  "term_id": "UNKNOWN:0002"
}